{
  "term_id": "GO:0008574",
  "term_label": "plus-end-directed microtubule motor activity",
  "gene_name": "Kinesin-like protein KIF16B",
  "gene": "UniProtKB:Q96L93",
  "gene_symbol": "KIF16B"
}